{
  "gene": "UniProtKB:Q06203",
  "gene_name": "Amidophosphoribosyltransferase",
  "term_id": "GO:0004044",
  "term_label": "amidophosphoribosyltransferase activity",
  "gene_symbol": "PPAT"
}